{
  "term_label": "Golgi membrane",
  "gene_symbol": "B3GALT1",
  "gene_name": "Beta-1,3-galactosyltransferase 1",
  "term_id": "GO:0000139",
  "gene": "UniProtKB:Q9Y5Z6"
}